{
  "gene_symbol": "Q6ZSR6",
  "gene_name": "Putative uncharacterized protein FLJ45256",
  "gene": "UniProtKB:Q6ZSR6",
  "term_id": "UNKNOWN:0003",
  "term_label": "Unknown cellular component"
}